{
  "gene_name": "Bromodomain-containing protein 1",
  "gene": "UniProtKB:O95696",
  "term_label": "chromatin remodeling",
  "term_id": "GO:0006338",
  "gene_symbol": "BRD1"
}